{
  "term_label": "microtubule organizing center",
  "gene_symbol": "SPECC1L",
  "gene": "UniProtKB:Q69YQ0",
  "term_id": "GO:0005815",
  "gene_name": "Cytospin-A"
}